{
  "gene": "UniProtKB:O94992",
  "gene_name": "Protein HEXIM1",
  "term_label": "negative regulation of transcription by RNA polymerase II",
  "gene_symbol": "HEXIM1",
  "term_id": "GO:0000122"
}